{
  "gene": "UniProtKB:O14520",
  "term_id": "GO:0015204",
  "term_label": "urea transmembrane transporter activity",
  "gene_symbol": "AQP7",
  "gene_name": "Aquaporin-7"
}